regulation of focal adhesion disassembly [GO:0120182] (biological process) Relationships: is a type of regulation of cell-substrate junction organization [GO:0150116]; regulates focal adhesion disassembly [GO:0120181] Subtypes: positive regulation of focal adhesion disassembly [GO:0120183], negative regulation of focal adhesion disassembly [GO:0120184] References: PMID:25490267 Definition: Any process that modulates the frequency, rate or extent of disaggregation of a focal adhesion into its constituent components.